{
  "gene_symbol": "RANBP1",
  "term_label": "nuclear pore",
  "gene": "UniProtKB:P43487",
  "gene_name": "Ran-specific GTPase-activating protein",
  "term_id": "GO:0005643"
}